{
  "term_label": "homotypic cell-cell adhesion",
  "gene_name": "CD99 antigen",
  "gene": "UniProtKB:P14209",
  "gene_symbol": "CD99",
  "term_id": "GO:0034109"
}